ovarian follicle endowment [GO:0001551] (biological process) Definition: Association of oocytes with supporting epithelial granulosa cells to form primordial follicles. References: PMID:30010832 Relationships: is a type of ovulation cycle process [GO:0022602]; is part of ovarian follicle development [GO:0001541]